ditrans, polycis-undecaprenyl-phosphate mannosyltransferase activity [GO:0036426] (molecular function) Definition: Catalysis of the reaction: ditrans,octacis-undecaprenyl phosphate + GDP-alpha-D-mannose = D-mannosyl undecaprenyl phosphate+ GDP. Sources: GOC:curators Relationships: is a type of undecaprenyl-phosphate mannosyltransferase activity [GO:0047267]